{
  "term_label": "high-affinity lysine transmembrane transporter activity",
  "term_id": "GO:0005292",
  "gene_name": "Mitochondrial basic amino acids transporter",
  "gene_symbol": "SLC25A29",
  "gene": "UniProtKB:Q8N8R3"
}